{
  "gene": "UniProtKB:Q8WU39",
  "gene_name": "Marginal zone B- and B1-cell-specific protein",
  "gene_symbol": "MZB1",
  "term_label": "endoplasmic reticulum chaperone complex",
  "term_id": "GO:0034663"
}